gastric acid secretion [GO:0001696] (biological process) Subtypes: GO:0001697, gastrin-induced gastric acid secretion [GO:0001698], acetylcholine-induced gastric acid secretion [GO:0001699] Regulation: regulated by GO:0060453; positively regulated by positive regulation of gastric acid secretion [GO:0060454]; negatively regulated by GO:0060455 Sources: GOC:hjd Also known as: hydrochloric acid secretion Definition: The regulated release of gastric acid (hydrochloric acid) by parietal or oxyntic cells during digestion. Relationships: is a type of GO:0022600; is a type of acid secretion [GO:0046717]